4-oxalocrotonate decarboxylase activity [GO:0047437] (molecular function) Sources: EC:4.1.1.77, MetaCyc:4.1.1.77-RXN Also known as: 4-oxalocrotonate carboxy-lyase (2-oxopent-4-enoate-forming), 4-oxalocrotonate carboxy-lyase activity Definition: Catalysis of the reaction: 4-oxalocrotonate = CO2 + 2-oxopent-4-enoate. Relationships: is a type of carboxy-lyase activity [GO:0016831]